{
  "gene": "UniProtKB:O00291",
  "term_id": "GO:2000588",
  "gene_symbol": "HIP1",
  "term_label": "positive regulation of platelet-derived growth factor receptor-beta signaling pathway",
  "gene_name": "Huntingtin-interacting protein 1"
}